synaptic vesicle, recycling pool [GO:1990475] (CC) Relationships: is a type of synaptic vesicle [GO:0008021]; is part of postsynapse [GO:0098794] Also known as: recycling pool of synaptic vesicles Definition: A synaptic vesicle belonging to the pool that repopulate vacancies within the readily releasable pool (RRP) of synaptic vesicles, and require more significant stimuli than the RRP in order to release neurotransmitter; about 10-15% of the total number of synaptic vesicles at a resting terminal bouton are in this state. References: PMID:22745285 Sources: GOC:pad